cerebellar granular layer structural organization [GO:0021685] (biological process) Also known as: cerebellar granular layer structural organisation Sources: GOC:cls, GOC:dgh, GOC:dph, GOC:jid, GO_REF:0000021 Relationships: is a type of anatomical structure arrangement [GO:0048532]; is part of cerebellar granular layer morphogenesis [GO:0021683]; is part of cerebellar cortex structural organization [GO:0021698] Definition: The process that contributes to the act of creating the structural organization of the cerebellar granule layer. This process pertains to the physical shaping of a rudimentary structure. The granular layer is the innermost layer of the cerebellar cortex. This layer contains densely packed small neurons, mostly granule cells. Some Golgi cells are found at the outer border. Granule neurons send parallel fibers to the upper molecular layer, where they synapse with Purkinje cell dendrites. Mossy fibers from the pontine nuclei in the white matter synapse with granule cell axons, Golgi cell axons and unipolar brush interneuron axons at cerebellar glomeruli in the granule cell layer.